negative regulation of vascular associated smooth muscle cell proliferation [GO:1904706] (biological process) Definition: Any process that stops, prevents or reduces the frequency, rate or extent of vascular smooth muscle cell proliferation. Relationships: is a type of negative regulation of smooth muscle cell proliferation [GO:0048662]; is a type of regulation of vascular associated smooth muscle cell proliferation [GO:1904705]; negatively regulates vascular associated smooth muscle cell proliferation [GO:1990874] References: PMID:23246467 Sources: GOC:TermGenie, GO_REF:0000058 Also known as: down regulation of VSMC proliferation, down regulation of vascular smooth muscle cell proliferation, down-regulation of VSMC proliferation, down-regulation of vascular smooth muscle cell proliferation, downregulation of VSMC proliferation, downregulation of vascular smooth muscle cell proliferation, negative regulation of VSMC proliferation, negative regulation of vascular smooth muscle cell proliferation, inhibition of VSMC proliferation, inhibition of vascular smooth muscle cell proliferation